positive regulation of voltage-gated potassium channel activity [GO:1903818] (biological process) Definition: Any process that activates or increases the frequency, rate or extent of voltage-gated potassium channel activity. References: PMID:19219384 Sources: GOC:TermGenie, GO_REF:0000059 Relationships: is a type of positive regulation of cation channel activity [GO:2001259]; positively regulates voltage-gated potassium channel activity [GO:0005249] Also known as: positive regulation of voltage gated potassium channel activity, positive regulation of voltage-dependent potassium channel activity, positive regulation of voltage-gated potassium ion channel activity, positive regulation of voltage-sensitive potassium channel, up regulation of voltage gated potassium channel activity, up regulation of voltage-dependent potassium channel activity, up regulation of voltage-gated potassium channel activity, up regulation of voltage-gated potassium ion channel activity, up regulation of voltage-sensitive potassium channel, up-regulation of voltage gated potassium channel activity, up-regulation of voltage-dependent potassium channel activity, up-regulation of voltage-gated potassium channel activity, up-regulation of voltage-gated potassium ion channel activity, up-regulation of voltage-sensitive potassium channel, upregulation of voltage gated potassium channel activity, upregulation of voltage-dependent potassium channel activity, upregulation of voltage-gated potassium channel activity, upregulation of voltage-gated potassium ion channel activity, upregulation of voltage-sensitive potassium channel, activation of voltage gated potassium channel activity, activation of voltage-dependent potassium channel activity, activation of voltage-gated potassium channel activity, activation of voltage-gated potassium ion channel activity, activation of voltage-sensitive potassium channel